{
  "gene": "UniProtKB:A6NML5",
  "gene_name": "Transmembrane protein 212",
  "gene_symbol": "TMEM212",
  "term_label": "Unknown biological process",
  "term_id": "UNKNOWN:0002"
}